positive regulation of endocytosis [GO:0045807] (biological process) Relationships: is a type of regulation of endocytosis [GO:0030100]; is a type of positive regulation of transport [GO:0051050]; is a type of positive regulation of cellular component organization [GO:0051130]; positively regulates endocytosis [GO:0006897] Definition: Any process that activates or increases the frequency, rate or extent of endocytosis. Sources: GOC:go_curators Subtypes: positive regulation of receptor-mediated endocytosis [GO:0048260], positive regulation of pinocytosis [GO:0048549], positive regulation of phagocytosis [GO:0050766], GO:1900244, positive regulation of ubiquitin-dependent endocytosis [GO:2000397], positive regulation of caveolin-mediated endocytosis [GO:2001288] Also known as: up regulation of endocytosis, up-regulation of endocytosis, upregulation of endocytosis, activation of endocytosis, stimulation of endocytosis